{
  "term_id": "GO:0005615",
  "term_label": "extracellular space",
  "gene_symbol": "APLN",
  "gene": "UniProtKB:Q9ULZ1",
  "gene_name": "Apelin"
}